{
  "gene_symbol": "LINGO1",
  "gene": "UniProtKB:Q96FE5",
  "term_id": "GO:0038023",
  "gene_name": "Leucine-rich repeat and immunoglobulin-like domain-containing nogo receptor-interacting protein 1",
  "term_label": "signaling receptor activity"
}